{
  "gene_symbol": "ABHD5",
  "gene": "UniProtKB:Q8WTS1",
  "term_id": "GO:0010898",
  "term_label": "positive regulation of triglyceride catabolic process",
  "gene_name": "1-acylglycerol-3-phosphate O-acyltransferase ABHD5"
}